{
  "term_id": "GO:0005665",
  "gene_symbol": "POLR2K",
  "term_label": "RNA polymerase II, core complex",
  "gene_name": "DNA-directed RNA polymerases I, II, and III subunit RPABC4",
  "gene": "UniProtKB:P53803"
}